L-gulonolactone oxidase activity [GO:0050105] (molecular function) Also known as: GLO activity, L-gulono-1,4-lactone:oxygen 3-oxidoreductase activity, L-gulono-gamma-lactone oxidase activity, L-gulono-gamma-lactone:O2 oxidoreductase activity, L-gulono-gamma-lactone:oxidoreductase activity Relationships: is a type of oxidoreductase activity, acting on the CH-OH group of donors, oxygen as acceptor [GO:0016899] Sources: EC:1.1.3.8, MetaCyc:L-GULONOLACTONE-OXIDASE-RXN, RHEA:32363 Definition: Catalysis of the reaction: L-gulono-1,4-lactone + O2 = L-xylo-hex-3-ulonolactone + H2O2.